regulation of translational frameshifting [GO:2001124] (biological process) Subtypes: negative regulation of translational frameshifting [GO:2001125], positive regulation of translational frameshifting [GO:2001126] Sources: GOC:obol Definition: Any process that modulates the frequency, rate or extent of translational frameshifting. Relationships: is a type of regulation of translational elongation [GO:0006448]; regulates translational frameshifting [GO:0006452]